{
  "gene_symbol": "SEMA4C",
  "gene": "UniProtKB:Q9C0C4",
  "term_id": "GO:0071526",
  "gene_name": "Semaphorin-4C",
  "term_label": "semaphorin-plexin signaling pathway"
}